{
  "gene": "UniProtKB:Q15046",
  "term_id": "GO:0002276",
  "term_label": "basophil activation involved in immune response",
  "gene_name": "Lysine--tRNA ligase",
  "gene_symbol": "KARS1"
}